Schwann cell proliferation involved in axon regeneration [GO:0014011] (biological process) Regulation: regulated by regulation of Schwann cell proliferation involved in axon regeneration [GO:1905044]; negatively regulated by negative regulation of Schwann cell proliferation involved in axon regeneration [GO:1905045]; positively regulated by positive regulation of Schwann cell proliferation involved in axon regeneration [GO:1905046] Sources: GOC:ef, ISBN:0878932585 Definition: The multiplication or reproduction of Schwann cells by cell division, resulting in the expansion of their population in response to an axonal lesion. The newly generated Schwann cells support subsequent axon regeneration in the peripheral nervous system. Relationships: is a type of Schwann cell proliferation [GO:0014010]; is part of GO:0014012